{
  "gene_symbol": "BCL2L13",
  "gene": "UniProtKB:Q9BXK5",
  "term_id": "GO:0005739",
  "term_label": "mitochondrion",
  "gene_name": "Bcl-2-like protein 13"
}